{
  "gene_symbol": "GDF6",
  "gene": "UniProtKB:Q6KF10",
  "term_label": "BMP signaling pathway",
  "gene_name": "Growth_differentiation factor 6",
  "term_id": "GO:0030509"
}